{
  "term_label": "intracellular sodium-activated potassium channel activity",
  "gene_name": "Potassium channel subfamily T member 2",
  "gene_symbol": "KCNT2",
  "term_id": "GO:0005228",
  "gene": "UniProtKB:Q6UVM3"
}